(R)-limonene synthase activity [GO:0034002] (molecular function) Sources: EC:4.2.3.20, RHEA:10940 Also known as: (+)-limonene synthase activity, geranyl-diphosphate diphosphate-lyase [cyclizing, (+)-(4R)-limonene-forming] activity, geranyldiphosphate diphosphate lyase [(+)-(R)-limonene-forming] activity Definition: Catalysis of the reaction: geranyl diphosphate = (4R)-limonene + diphosphate. Relationships: is a type of GO:0010333